germ cell development [GO:0007281] (biological process) Sources: GOC:go_curators Also known as: germ-cell development, gametogenesis, primordial germ cell development Definition: The process whose specific outcome is the progression of an immature germ cell over time, from its formation to the mature structure (gamete). A germ cell is any reproductive cell in a multicellular organism. Relationships: is a type of developmental process involved in reproduction [GO:0003006]; is a type of cellular process involved in reproduction in multicellular organism [GO:0022412]; is a type of cell development [GO:0048468]; is part of gamete generation [GO:0007276] Subtypes: spermatid development [GO:0007286], oogenesis [GO:0048477], oocyte development [GO:0048599]